{
  "term_id": "GO:0005886",
  "term_label": "plasma membrane",
  "gene_name": "Urotensin-2 receptor",
  "gene_symbol": "UTS2R",
  "gene": "UniProtKB:Q9UKP6"
}